{
  "gene": "UniProtKB:P00441",
  "term_label": "cytosol",
  "term_id": "GO:0005829",
  "gene_symbol": "SOD1",
  "gene_name": "Superoxide dismutase [Cu-Zn]"
}